{
  "gene_name": "NACHT, LRR and PYD domains-containing protein 12",
  "term_label": "negative regulation of canonical NF-kappaB signal transduction",
  "gene": "UniProtKB:P59046",
  "term_id": "GO:0043124",
  "gene_symbol": "NLRP12"
}